{
  "gene_symbol": "SYNPO2",
  "gene_name": "Synaptopodin-2",
  "term_label": "positive regulation of actin filament bundle assembly",
  "term_id": "GO:0032233",
  "gene": "UniProtKB:Q9UMS6"
}